{
  "gene_symbol": "PDLIM7",
  "gene": "UniProtKB:Q9NR12",
  "term_id": "GO:0030018",
  "gene_name": "PDZ and LIM domain protein 7",
  "term_label": "Z disc"
}